{
  "gene_symbol": "KNTC1",
  "gene": "UniProtKB:P50748",
  "gene_name": "Kinetochore-associated protein 1",
  "term_id": "GO:1990423",
  "term_label": "RZZ complex"
}